{
  "gene": "UniProtKB:O75937",
  "gene_symbol": "DNAJC8",
  "term_label": "Unknown molecular function",
  "term_id": "UNKNOWN:0001",
  "gene_name": "DnaJ homolog subfamily C member 8"
}